{
  "term_id": "GO:0043162",
  "term_label": "ubiquitin-dependent protein catabolic process via the multivesicular body sorting pathway",
  "gene_name": "Ubiquitin-associated protein 1",
  "gene": "UniProtKB:Q9NZ09",
  "gene_symbol": "UBAP1"
}